{
  "term_id": "GO:0090162",
  "gene_symbol": "SIPA1L3",
  "gene_name": "Signal-induced proliferation-associated 1-like protein 3",
  "gene": "UniProtKB:O60292",
  "term_label": "establishment of epithelial cell polarity"
}